formation of a compartment boundary [GO:0060288] (biological process) Definition: Formation of a lineage restriction boundary within a developing tissue which does not correspond to some morphological barrier. Sources: GOC:dph Relationships: is a type of GO:0048859; is part of compartment pattern specification [GO:0007386] Also known as: compartment boundary formation